vacuole organization [GO:0007033] (biological process) Also known as: vacuole organisation, vacuolar assembly, vacuole biogenesis, vacuole organization and biogenesis Regulation: regulated by regulation of vacuole organization [GO:0044088]; positively regulated by positive regulation of vacuole organization [GO:0044090] Subtypes: vacuole inheritance [GO:0000011], contractile vacuole organization [GO:0033298], notochord cell vacuolation [GO:0060036], lytic vacuole organization [GO:0080171], GO:0097576, autophagosome organization [GO:1905037], GO:1990019 Definition: A process that is carried out at the cellular level which results in the assembly, arrangement of constituent parts, or disassembly of a vacuole. Relationships: is a type of organelle organization [GO:0006996] Sources: GOC:mah